vibriobactin metabolic process [GO:0019536] (BP) Definition: The chemical reactions and pathways involving vibriobactin, the major siderophore produced by Vibrio cholerae. References: PMID:11112537 Sources: GOC:jl Also known as: vibriobactin metabolism Relationships: is a type of GO:0009237; is a type of amide metabolic process [GO:0043603] Subtypes: GO:0019537